{
  "term_label": "trans-Golgi network",
  "gene": "UniProtKB:Q8IUQ0",
  "gene_name": "Clavesin-1",
  "gene_symbol": "CLVS1",
  "term_id": "GO:0005802"
}